{
  "gene_symbol": "TRNAU1AP",
  "term_id": "GO:0005634",
  "gene_name": "tRNA selenocysteine 1-associated protein 1",
  "term_label": "nucleus",
  "gene": "UniProtKB:Q9NX07"
}